ABC-type bacteriocin transporter activity [GO:0043214] (MF) Definition: Enables the transfer of a bacteriocin from one side of a membrane to the other according to the reaction: ATP + H2O = ADP + phosphate. References: PMID:33040342 Sources: GOC:mlg Also known as: ABC-type bacteriocin transmembrane transporter activity, bacteriocin ABC transporter, ATPase-coupled bacteriocin transmembrane transporter activity Relationships: is a type of ABC-type xenobiotic transporter activity [GO:0008559]; is_a GO:0022885